{
  "gene": "UniProtKB:Q6ZUX3",
  "term_id": "GO:0005929",
  "term_label": "cilium",
  "gene_symbol": "TOGARAM2",
  "gene_name": "TOG array regulator of axonemal microtubules protein 2"
}